{
  "term_id": "GO:0000981",
  "term_label": "DNA-binding transcription factor activity, RNA polymerase II-specific",
  "gene": "UniProtKB:Q92988",
  "gene_symbol": "DLX4",
  "gene_name": "Homeobox protein DLX-4"
}